{
  "gene_name": "KN motif and ankyrin repeat domain-containing protein 1",
  "term_label": "negative regulation of actin filament polymerization",
  "gene": "UniProtKB:Q14678",
  "term_id": "GO:0030837",
  "gene_symbol": "KANK1"
}